RNA exonuclease activity, producing 5'-phosphomonoesters [GO:0016896] (molecular function) Sources: GOC:ai Relationships: is a type of GO:0004532 Subtypes: 3'-5'-RNA exonuclease activity [GO:0000175], exoribonuclease H activity [GO:0004533], GO:0004534, GO:0033890 Also known as: exoribonuclease activity, producing 5' phosphomonoesters, exoribonuclease activity, producing 5'-phosphomonoesters Definition: Catalysis of the hydrolysis of ester linkages within ribonucleic acids by removing nucleotide residues from the 3' or 5' end to yield 5' phosphomonoesters.